{
  "term_label": "cell surface",
  "gene_name": "Neurogenic locus notch homolog protein 1",
  "gene_symbol": "NOTCH1",
  "term_id": "GO:0009986",
  "gene": "UniProtKB:P46531"
}